{
  "gene": "UniProtKB:A6NHM9",
  "gene_name": "Putative DBH-like monooxygenase protein 2",
  "term_label": "secretory granule membrane",
  "gene_symbol": "MOXD2P",
  "term_id": "GO:0030667"
}